{
  "gene_name": "Uncharacterized protein C10orf67, mitochondrial",
  "gene_symbol": "C10orf67",
  "gene": "UniProtKB:Q8IYJ2",
  "term_id": "UNKNOWN:0003",
  "term_label": "Unknown cellular component"
}